{
  "term_id": "GO:0005815",
  "gene": "UniProtKB:Q6P9F0",
  "gene_symbol": "CCDC62",
  "gene_name": "Coiled-coil domain-containing protein 62",
  "term_label": "microtubule organizing center"
}